{
  "term_id": "GO:0005789",
  "gene_name": "Homocysteine-responsive endoplasmic reticulum-resident ubiquitin-like domain member 1 protein",
  "gene_symbol": "HERPUD1",
  "gene": "UniProtKB:Q15011",
  "term_label": "endoplasmic reticulum membrane"
}